synaptic transmission, GABAergic [GO:0051932] (biological process) Regulation: regulated by regulation of synaptic transmission, GABAergic [GO:0032228]; negatively regulated by negative regulation of synaptic transmission, GABAergic [GO:0032229]; positively regulated by GO:0032230 Definition: The vesicular release of gamma-aminobutyric acid (GABA). from a presynapse, across a chemical synapse, the subsequent activation of GABA receptors at the postsynapse of a target cell (neuron, muscle, or secretory cell) and the effects of this activation on the postsynaptic membrane potential and ionic composition of the postsynaptic cytosol. This process encompasses both spontaneous and evoked release of neurotransmitter and all parts of synaptic vesicle exocytosis. Evoked transmission starts with the arrival of an action potential at the presynapse. Sources: GOC:dos, ISBN:0126603030 Relationships: is_a chemical synaptic transmission [GO:0007268] Also known as: GABAergic synaptic transmission, synaptic transmission, GABA mediated, synaptic transmission, gamma-aminobutyric acid mediated, synaptic transmission, gamma-aminobutyric acid-ergic